{
  "gene_name": "Pumilio homolog 1",
  "gene": "UniProtKB:Q14671",
  "term_label": "cytoplasm",
  "gene_symbol": "PUM1",
  "term_id": "GO:0005737"
}